{
  "gene_symbol": "SMIM1",
  "gene": "UniProtKB:B2RUZ4",
  "gene_name": "Small integral membrane protein 1",
  "term_label": "plasma membrane",
  "term_id": "GO:0005886"
}